{
  "term_id": "GO:0006702",
  "gene_name": "3-oxo-5-alpha-steroid 4-dehydrogenase 2",
  "term_label": "androgen biosynthetic process",
  "gene_symbol": "SRD5A2",
  "gene": "UniProtKB:P31213"
}